{
  "gene_name": "SLIT-ROBO Rho GTPase-activating protein 2C",
  "term_id": "GO:0007399",
  "gene": "UniProtKB:P0DJJ0",
  "term_label": "nervous system development",
  "gene_symbol": "SRGAP2C"
}